{
  "gene_name": "Proteasome subunit alpha type-4",
  "term_label": "nucleus",
  "gene": "UniProtKB:P25789",
  "term_id": "GO:0005634",
  "gene_symbol": "PSMA4"
}